development of primary female sexual characteristics [GO:0046545] (biological process) Definition: The process whose specific outcome is the progression of the primary female sexual characteristics over time, from their formation to the mature structure. The primary female sexual characteristics are the ovaries, and they develop in response to sex hormone secretion. Sources: GOC:ai Relationships: is a type of development of primary sexual characteristics [GO:0045137]; is part of female sex differentiation [GO:0046660]